{
  "term_label": "homophilic cell-cell adhesion",
  "gene_name": "Pregnancy-specific beta-1-glycoprotein 2",
  "gene": "UniProtKB:P11465",
  "gene_symbol": "PSG2",
  "term_id": "GO:0007156"
}